{
  "gene_symbol": "BTBD3",
  "gene_name": "BTB_POZ domain-containing protein 3",
  "term_label": "cytosol",
  "gene": "UniProtKB:Q9Y2F9",
  "term_id": "GO:0005829"
}